{
  "gene_name": "Condensin-2 complex subunit G2",
  "gene_symbol": "NCAPG2",
  "gene": "UniProtKB:Q86XI2",
  "term_id": "GO:0000070",
  "term_label": "mitotic sister chromatid segregation"
}